{
  "gene_name": "Microtubule cross-linking factor 1",
  "gene": "UniProtKB:Q9Y4B5",
  "term_label": "microtubule binding",
  "gene_symbol": "MTCL1",
  "term_id": "GO:0008017"
}